{
  "gene_name": "Unconventional myosin-Vc",
  "term_label": "membrane",
  "term_id": "GO:0016020",
  "gene": "UniProtKB:Q9NQX4",
  "gene_symbol": "MYO5C"
}